cellular response to external biotic stimulus [GO:0071217] (biological process) Relationships: is a type of GO:0043207; is a type of cellular response to biotic stimulus [GO:0071216]; is a type of cellular response to external stimulus [GO:0071496] Sources: GOC:mah Definition: Any process that results in a change in state or activity of a cell (in terms of movement, secretion, enzyme production, gene expression, etc.) as a result of an external biotic stimulus, an external stimulus caused by, or produced by living things.